{
  "term_label": "cytoplasm",
  "term_id": "GO:0005737",
  "gene": "UniProtKB:Q13131",
  "gene_name": "5'-AMP-activated protein kinase catalytic subunit alpha-1",
  "gene_symbol": "PRKAA1"
}